{
  "gene": "UniProtKB:Q96BY9",
  "gene_name": "Store-operated calcium entry-associated regulatory factor",
  "term_id": "GO:2001256",
  "gene_symbol": "SARAF",
  "term_label": "regulation of store-operated calcium entry"
}